{
  "term_id": "UNKNOWN:0001",
  "term_label": "Unknown molecular function",
  "gene_symbol": "MICOS10",
  "gene_name": "MICOS complex subunit MIC10",
  "gene": "UniProtKB:Q5TGZ0"
}